butirosin biosynthetic process [GO:1901758] (biological process) Definition: The chemical reactions and pathways resulting in the formation of butirosin. Also known as: butirosin anabolism, butirosin biosynthesis, butirosin formation, butirosin synthesis Relationships: is a type of GO:0016138; is a type of polyol biosynthetic process [GO:0046173] Sources: GOC:TermGenie, GOC:yaf, UniPathway:UPA00964